tryptophan alpha,beta-oxidase activity [GO:0050621] (molecular function) Also known as: tryptophan a,b-oxidase activity, L-tryptophan 2',3'-oxidase activity, L-tryptophan alpha,beta-dehydrogenase activity, L-tryptophan:oxygen alpha,beta-oxidoreductase activity Sources: EC:1.3.3.10, RHEA:19901 Note: Note that this was EC:1.4.3.17. Relationships: is a type of GO:0016634 Definition: Catalysis of the reaction: L-tryptophan + O2 = alpha,beta-didehydrotryptophan + H2O2 + H+.